{
  "gene_name": "Uncharacterized protein C10orf95",
  "gene": "UniProtKB:Q9H7T3",
  "gene_symbol": "C10orf95",
  "term_id": "UNKNOWN:0001",
  "term_label": "Unknown molecular function"
}